{
  "term_id": "GO:0007166",
  "term_label": "cell surface receptor signaling pathway",
  "gene": "UniProtKB:A0A5B0",
  "gene_symbol": "TRBV14",
  "gene_name": "T cell receptor beta variable 14"
}